{
  "term_id": "GO:0005594",
  "gene_name": "Collagen alpha-1(IX) chain",
  "gene": "UniProtKB:P20849",
  "term_label": "collagen type IX trimer",
  "gene_symbol": "COL9A1"
}